negative regulation of wound healing, spreading of epidermal cells [GO:1903690] (biological process) Definition: Any process that stops, prevents or reduces the frequency, rate or extent of wound healing, spreading of epidermal cells. References: PMID:18394891 Sources: GOC:TermGenie, GOC:als, GO_REF:0000058 Also known as: down regulation of wound healing, spreading of epidermal cells, down-regulation of wound healing, spreading of epidermal cells, downregulation of wound healing, spreading of epidermal cells, inhibition of wound healing, spreading of epidermal cells Relationships: is a type of negative regulation of cell migration [GO:0030336]; is a type of GO:0061045; is a type of regulation of wound healing, spreading of epidermal cells [GO:1903689]; negatively regulates wound healing, spreading of epidermal cells [GO:0035313]